{
  "gene": "UniProtKB:A8MU10",
  "term_label": "Unknown molecular function",
  "term_id": "UNKNOWN:0001",
  "gene_name": "Putative uncharacterized protein ENSP00000381562",
  "gene_symbol": "A8MU10"
}